glucosylglycerate hydrolase activity [GO:0102547] (molecular function) Definition: Catalysis of the reaction: (2R)-2-O-(alpha-D-glucopyranosyl)-glycerate + H2O = (R)-glycerate + D-glucose. Sources: RHEA:32059 Relationships: is a type of GO:0016803